single-stranded DNA endodeoxyribonuclease activity [GO:0000014] (molecular function) Also known as: single-stranded DNA specific endodeoxyribonuclease activity, ssDNA-specific endodeoxyribonuclease activity Definition: Catalysis of the hydrolysis of ester linkages within a single-stranded deoxyribonucleic acid molecule by creating internal breaks. Subtypes: 3' overhang single-stranded DNA endodeoxyribonuclease activity [GO:1990599], GO:1990601 Sources: GOC:mah Regulation: positively regulated by single-stranded DNA endodeoxyribonuclease activator activity [GO:1990600] Relationships: is a type of GO:0004520; is_a hydrolase activity, acting on ester bonds [GO:0016788]